vasculogenesis involved in coronary vascular morphogenesis [GO:0060979] (biological process) Also known as: coronary vasculogenesis, vasculogenesis involved in coronary blood vessel morphogenesis Relationships: is a type of vasculogenesis [GO:0001570]; is part of coronary vasculature morphogenesis [GO:0060977] Definition: The differentiation of endothelial cells from progenitor cells that contributes to blood vessel development in the heart, and the de novo formation of blood vessels and tubes. Sources: GOC:mtg_heart